{
  "gene": "UniProtKB:Q9Y2A7",
  "term_label": "cortical actin cytoskeleton organization",
  "gene_name": "Nck-associated protein 1",
  "gene_symbol": "NCKAP1",
  "term_id": "GO:0030866"
}